{
  "gene_name": "Peroxiredoxin-1",
  "gene_symbol": "PRDX1",
  "term_label": "removal of superoxide radicals",
  "term_id": "GO:0019430",
  "gene": "UniProtKB:Q06830"
}